intracellular receptor signaling pathway [GO:0030522] (biological process) Also known as: intracellular receptor mediated signaling pathway, intracellular receptor-mediated signaling pathway, intracellular receptor-mediated signalling pathway Sources: GOC:bf, GOC:mah Definition: The series of molecular signals initiated by a ligand binding to a receptor located within a cell. Subtypes: cytoplasmic pattern recognition receptor signaling pathway [GO:0002753], GO:0009785, juvenile hormone mediated signaling pathway [GO:0035626], nuclear receptor-mediated signaling pathway [GO:0141193] Relationships: is_a intracellular signal transduction [GO:0035556]